{
  "term_label": "Unknown biological process",
  "term_id": "UNKNOWN:0002",
  "gene_symbol": "VN1R17P",
  "gene": "UniProtKB:Q8TDU5",
  "gene_name": "Putative vomeronasal receptor-like protein 4"
}